{
  "gene_symbol": "TMEM132B",
  "gene_name": "Transmembrane protein 132B",
  "term_id": "GO:0016020",
  "gene": "UniProtKB:Q14DG7",
  "term_label": "membrane"
}